nuclear mRNA surveillance of spliceosomal pre-mRNA splicing [GO:0071030] (biological process) Relationships: is a type of nuclear mRNA surveillance [GO:0071028]; has part nuclear polyadenylation-dependent mRNA catabolic process [GO:0071042] References: PMID:18644474 Sources: GOC:dgf, GOC:krc Also known as: nuclear RNA catabolic process of incorrectly spliced pre-mRNA, nuclear mRNA quality control of incorrectly spliced pre-mRNA Definition: The set of processes involved in identifying and degrading incorrectly spliced pre-mRNAs within the nucleus.